TMEM240-body [GO:0160045] (cellular component) Relationships: is a type of intracellular membrane-bounded organelle [GO:0043231] Also known as: T240-body Definition: A multilamellar subcellular structure formed in the cytoplasm of developing neuron, composed of Tmem240 and Emd proteins. References: PMID:32535204